{
  "gene_symbol": "APOBEC3H",
  "term_id": "GO:0003723",
  "gene": "UniProtKB:Q6NTF7",
  "term_label": "RNA binding",
  "gene_name": "DNA dC-dU-editing enzyme APOBEC-3H"
}